regulation of stomach fundus smooth muscle contraction [GO:0120068] (biological process) Definition: Any process that modulates the frequency, rate or extent of any stomach fundus smooth muscle contraction. References: PMID:15890336 Sources: GOC:sl Relationships: is a type of GO:1904304; regulates stomach fundus smooth muscle contraction [GO:0014825] Subtypes: positive regulation of stomach fundus smooth muscle contraction [GO:0120069], negative regulation of stomach fundus smooth muscle contraction [GO:0120070]